FMN reductase (NADPH) activity [GO:0052873] (MF) Relationships: is a type of FMN reductase [NAD(P)H] activity [GO:0008752] Sources: RHEA:21624 Definition: Catalysis of the reaction: FMNH2 + NADP+ = FMN + NADPH + 2 H+. Also known as: NADPH dehydrogenase (FMN) activity